purine ribonucleoside monophosphate biosynthetic process [GO:0009168] (biological process) Also known as: purine ribonucleoside monophosphate anabolism, purine ribonucleoside monophosphate biosynthesis, purine ribonucleoside monophosphate formation, purine ribonucleoside monophosphate synthesis Sources: GOC:go_curators, ISBN:0198506732 Definition: The chemical reactions and pathways resulting in the formation of purine ribonucleoside monophosphate, a compound consisting of a purine base linked to a ribose sugar esterified with phosphate on the sugar. Relationships: is a type of GO:0009127; is a type of ribonucleoside monophosphate biosynthetic process [GO:0009156]; is a type of GO:0009167 Subtypes: AMP biosynthetic process [GO:0006167], GMP biosynthetic process [GO:0006177], IMP biosynthetic process [GO:0006188], GO:0097293